{
  "term_id": "GO:0015269",
  "gene_symbol": "KCNMB3",
  "term_label": "calcium-activated potassium channel activity",
  "gene": "UniProtKB:Q9NPA1",
  "gene_name": "Calcium-activated potassium channel subunit beta-3"
}